positive regulation of glucuronoarabinoxylan catabolic process [GO:2000920] (biological process) Also known as: positive regulation of glucuronoarabinoxylan catabolism Relationships: is a type of positive regulation of glucuronoxylan catabolic process [GO:2000917]; is_a GO:2000918; is a type of positive regulation of arabinoxylan-containing compound catabolic process [GO:2000923]; RO_0002213 glucuronoarabinoxylan catabolic process [GO:2000887] Sources: GOC:mengo_curators Definition: Any process that activates or increases the frequency, rate or extent of glucuronoarabinoxylan catabolic process.